{
  "gene": "UniProtKB:Q9Y2Y4",
  "gene_name": "Zinc finger and BTB domain-containing protein 32",
  "term_id": "GO:0002682",
  "term_label": "regulation of immune system process",
  "gene_symbol": "ZBTB32"
}